{
  "term_id": "GO:0080008",
  "gene_symbol": "DCAF10",
  "term_label": "Cul4-RING E3 ubiquitin ligase complex",
  "gene_name": "DDB1- and CUL4-associated factor 10",
  "gene": "UniProtKB:Q5QP82"
}